{
  "term_id": "GO:0032991",
  "gene_name": "Heat shock protein HSP 90-beta",
  "gene_symbol": "HSP90AB1",
  "term_label": "protein-containing complex",
  "gene": "UniProtKB:P08238"
}